{
  "gene": "UniProtKB:Q96IT1",
  "gene_name": "Zinc finger protein 496",
  "term_id": "GO:0006357",
  "gene_symbol": "ZNF496",
  "term_label": "regulation of transcription by RNA polymerase II"
}